(+)-beta-chamigrene synthase activity [GO:0102883] (molecular function) Sources: RHEA:30379 Relationships: is a type of GO:0016838 Definition: Catalysis of the reaction: (2E,6E)-farnesyl diphosphate = (+)-beta-chamigrene + diphosphate.